{
  "gene": "UniProtKB:Q96NM4",
  "gene_name": "TOX high mobility group box family member 2",
  "term_label": "nucleus",
  "term_id": "GO:0005634",
  "gene_symbol": "TOX2"
}